NAD-dependent protein demyristoylase activity [GO:0140773] (molecular function) Relationships: is_a acyltransferase activity, transferring groups other than amino-acyl groups [GO:0016747]; is part of post-translational protein modification [GO:0043687] References: PMID:23552949 Sources: RHEA:70567 Definition: Catalysis of the reaction: N6-tetradecanoyl-L-lysyl-[protein] + NAD+ + H2O = tetradecanoyl-ADP-D-ribose + L-lysyl-[protein] + nicotinamide.